{
  "gene_name": "Sorting nexin-29",
  "term_id": "UNKNOWN:0003",
  "gene_symbol": "SNX29",
  "term_label": "Unknown cellular component",
  "gene": "UniProtKB:Q8TEQ0"
}